{
  "gene_name": "Tyrosine-protein kinase JAK1",
  "term_label": "intracellular signal transduction",
  "term_id": "GO:0035556",
  "gene_symbol": "JAK1",
  "gene": "UniProtKB:P23458"
}